8-oxocoformycin reductase activity [GO:0047599] (molecular function) Also known as: 8-ketodeoxycoformycin reductase activity, coformycin:NADP+ 8-oxidoreductase activity Relationships: is a type of oxidoreductase activity, acting on the CH-OH group of donors, NAD or NADP as acceptor [GO:0016616] Sources: EC:1.1.1.235, RHEA:23168 Definition: Catalysis of the reaction: coformycin + NADP+ = 8-oxocoformycin + 2 H+ + NADPH.